mycocerosate synthase activity [GO:0050111] (molecular function) Sources: EC:2.3.1.111, RHEA:10588 Relationships: is a type of GO:0016747 Definition: Catalysis of the reaction: acyl-CoA + 7n H+ + n methylmalonyl-CoA + 2n NADPH = n CO2 + n CoA + n H2O + multi-methyl-branched acyl-CoA + 2n NADP+. Also known as: acyl-CoA:methylmalonyl-CoA C-acyltransferase (decarboxylating, oxoacyl- and enoyl-reducing), mycocerosic acid synthase activity